{
  "term_label": "Unknown cellular component",
  "gene_name": "Zinc finger protein 215",
  "gene_symbol": "ZNF215",
  "term_id": "UNKNOWN:0003",
  "gene": "UniProtKB:Q9UL58"
}